postsynaptic specialization assembly [GO:0098698] (biological process) Definition: The aggregation, arrangement and bonding together of a set of components to form a postsynaptic specialization, a region that lies adjacent to the cytoplasmic face of the postsynaptic membrane. Sources: GOC:dos Relationships: is a type of organelle assembly [GO:0070925]; is a type of postsynaptic specialization organization [GO:0099084]; is part of postsynapse assembly [GO:0099068] Subtypes: postsynaptic density assembly [GO:0097107] Regulation: regulated by regulation of postsynaptic specialization assembly [GO:0099150]